{
  "gene_name": "Neurochondrin",
  "gene": "UniProtKB:Q9UBB6",
  "gene_symbol": "NCDN",
  "term_label": "regulation of neuronal synaptic plasticity",
  "term_id": "GO:0048168"
}